X11-like protein binding [GO:0042988] (molecular function) References: PMID:12780348 Sources: GOC:jl Definition: Binding to X11-like protein, a neuron-specific adaptor protein. Also known as: X11L binding Relationships: is_a GO:0005515